PAK family kinase-Sog2 complex [GO:0099125] (cellular component) Relationships: is a type of protein kinase complex [GO:1902911] References: PMID:23462181 Definition: A protein kinase complex comprising a conserved PAK/GC/Ste20 family kinase, leucine rich repeat protein Sog2 family, which function as part of the cell shape network.